(S)-scoulerine 9-O-methyltransferase activity [GO:0030777] (molecular function) Definition: Catalysis of the reaction: (S)-scoulerine + S-adenosyl-L-methionine(1+) = (S)-tetrahydrocolumbamine + S-adenosyl-L-homocysteine + H+. Also known as: S-adenosyl-L-methionine:(S)-scoclaurine 9-O-methyltransferase activity, S-adenosyl-L-methionine:(S)-scoulerine 9-O-methyltransferase activity Relationships: is a type of S-adenosylmethionine-dependent methyltransferase activity [GO:0008757] Sources: EC:2.1.1.117, RHEA:23808